{
  "gene_name": "FAST kinase domain-containing protein 2, mitochondrial",
  "term_id": "GO:0003723",
  "gene": "UniProtKB:Q9NYY8",
  "term_label": "RNA binding",
  "gene_symbol": "FASTKD2"
}